imaginal disc-derived wing hair outgrowth [GO:0035318] (biological process) Also known as: wing hair outgrowth, wing prehair outgrowth References: PMID:11064425, PMID:8947551 Sources: GOC:mtg_sensu Definition: Extrusion of a cellular projection from the apical membrane of an epithelial cell in an imaginal disc-derived wing. Outgrowth initiates approximately 35 hours after puparium formation from the distal side of the cell, and at this stage the cellular extension is termed a prehair. Relationships: is a type of post-embryonic animal morphogenesis [GO:0009886]; is a type of cell projection morphogenesis [GO:0048858]; is part of GO:0035317